{
  "term_id": "UNKNOWN:0003",
  "term_label": "Unknown cellular component",
  "gene_symbol": "IL27RA",
  "gene": "UniProtKB:Q6UWB1",
  "gene_name": "Interleukin-27 receptor subunit alpha"
}